{
  "term_label": "regulation of cardiac muscle contraction by regulation of the release of sequestered calcium ion",
  "gene_symbol": "FKBP1A",
  "gene_name": "Peptidyl-prolyl cis-trans isomerase FKBP1A",
  "term_id": "GO:0010881",
  "gene": "UniProtKB:P62942"
}